regulation of branch elongation involved in ureteric bud branching [GO:0072095] (biological process) Subtypes: negative regulation of branch elongation involved in ureteric bud branching [GO:0072096] Relationships: is a type of regulation of developmental growth [GO:0048638]; regulates branch elongation involved in ureteric bud branching [GO:0060681] Sources: GOC:mtg_kidney_jan10 Definition: Any process that modulates the frequency, rate or extent of branch elongation involved in ureteric bud branching, the growth of a branch of the ureteric bud along its axis.